positive regulation of interleukin-18-mediated signaling pathway [GO:2000494] (biological process) Sources: GOC:obol Also known as: positive regulation of interleukin-18-mediated signalling pathway Definition: Any process that activates or increases the frequency, rate or extent of interleukin-18-mediated signaling pathway. Relationships: is a type of positive regulation of cytokine-mediated signaling pathway [GO:0001961]; is a type of regulation of interleukin-18-mediated signaling pathway [GO:2000492]; RO_0002213 GO:0035655